{
  "gene_symbol": "FAM187B",
  "term_label": "Unknown biological process",
  "gene_name": "Protein FAM187B",
  "term_id": "UNKNOWN:0002",
  "gene": "UniProtKB:Q17R55"
}